phosphinothricin catabolic process [GO:1901765] (biological process) Sources: GOC:TermGenie, GOC:yaf Relationships: is a type of catabolic process [GO:0009056]; is a type of phosphinothricin metabolic process [GO:1901764] Definition: The chemical reactions and pathways resulting in the breakdown of phosphinothricin. Also known as: phosphinothricin breakdown, phosphinothricin catabolism, phosphinothricin degradation